{
  "gene_symbol": "MICAL2",
  "term_id": "GO:0005886",
  "gene": "UniProtKB:O94851",
  "term_label": "plasma membrane",
  "gene_name": "[F-actin]-monooxygenase MICAL2"
}